{
  "gene": "UniProtKB:Q8TC44",
  "gene_name": "POC1 centriolar protein homolog B",
  "term_label": "ciliary basal body",
  "term_id": "GO:0036064",
  "gene_symbol": "POC1B"
}